4-hydroxyproline biosynthetic process [GO:0019472] (biological process) Definition: The chemical reactions and pathways resulting in the formation of 4-hydroxyproline, C5H9NO3, a derivative of the amino acid proline. Sources: GOC:ai Also known as: 4-hydroxyproline anabolism, 4-hydroxyproline biosynthesis, 4-hydroxyproline formation, 4-hydroxyproline synthesis Relationships: is a type of GO:0042398; is a type of non-proteinogenic amino acid biosynthetic process [GO:0170043]; is a type of alpha-amino acid biosynthetic process [GO:1901607]